{
  "gene": "UniProtKB:Q8TAT5",
  "gene_symbol": "NEIL3",
  "term_label": "DNA-(apurinic or apyrimidinic site) endonuclease activity",
  "term_id": "GO:0003906",
  "gene_name": "Endonuclease 8-like 3"
}